{
  "term_id": "UNKNOWN:0003",
  "gene": "UniProtKB:Q9H9V4",
  "term_label": "Unknown cellular component",
  "gene_symbol": "RNF122",
  "gene_name": "RING finger protein 122"
}